{
  "term_id": "UNKNOWN:0003",
  "term_label": "Unknown cellular component",
  "gene_symbol": "TMEM217B",
  "gene": "UniProtKB:A0A494BZU4",
  "gene_name": "Putative transmembrane protein 217B"
}